amine binding [GO:0043176] (molecular function) Sources: GOC:jl Definition: Binding to an amine, a weakly basic organic compound that contains an amino or a substituted amino group. Subtypes: phenylalkylamine binding [GO:0008145], polyamine binding [GO:0019808], serotonin binding [GO:0051378], 1-(4-iodo-2,5-dimethoxyphenyl)propan-2-amine binding [GO:0071886] Relationships: is_a GO:0005488